{
  "gene_name": "Neurexin-1",
  "gene": "UniProtKB:Q9ULB1",
  "gene_symbol": "NRXN1",
  "term_id": "GO:0007399",
  "term_label": "nervous system development"
}